{
  "term_label": "chromatin remodeling",
  "gene_symbol": "PRMT2",
  "gene_name": "Protein arginine N-methyltransferase 2",
  "gene": "UniProtKB:P55345",
  "term_id": "GO:0006338"
}